{
  "gene_name": "Lipolysis-stimulated lipoprotein receptor",
  "gene": "UniProtKB:Q86X29",
  "term_id": "UNKNOWN:0001",
  "term_label": "Unknown molecular function",
  "gene_symbol": "LSR"
}